{
  "gene_name": "V-type proton ATPase subunit d 2",
  "term_label": "vacuolar transport",
  "gene": "UniProtKB:Q8N8Y2",
  "term_id": "GO:0007034",
  "gene_symbol": "ATP6V0D2"
}